{
  "term_id": "UNKNOWN:0001",
  "term_label": "Unknown molecular function",
  "gene": "UniProtKB:Q6ZRS4",
  "gene_name": "Protein ITPRID1",
  "gene_symbol": "ITPRID1"
}